{
  "gene": "UniProtKB:Q8TAA9",
  "term_id": "GO:0005886",
  "gene_name": "Vang-like protein 1",
  "term_label": "plasma membrane",
  "gene_symbol": "VANGL1"
}